{
  "gene_name": "HCG1807616",
  "gene": "UniProtKB:A0A1W2PRN6",
  "term_label": "RNA polymerase II general transcription initiation factor activity",
  "term_id": "GO:0016251",
  "gene_symbol": "LINC02218"
}